{
  "gene": "UniProtKB:Q9BZR9",
  "term_label": "Unknown molecular function",
  "gene_symbol": "TRIM8",
  "term_id": "UNKNOWN:0001",
  "gene_name": "E3 ubiquitin-protein ligase TRIM8"
}